{
  "gene": "UniProtKB:Q8IYB7",
  "term_label": "mRNA catabolic process",
  "gene_name": "DIS3-like exonuclease 2",
  "gene_symbol": "DIS3L2",
  "term_id": "GO:0006402"
}